clathrin light chain binding [GO:0032051] (molecular function) Definition: Binding to a clathrin light chain. Sources: GOC:mah Relationships: is a type of clathrin binding [GO:0030276]